regulation of hydrogen peroxide catabolic process [GO:2000295] (biological process) Subtypes: positive regulation of hydrogen peroxide catabolic process [GO:1903285], negative regulation of hydrogen peroxide catabolic process [GO:2000296] Sources: GOC:BHF Also known as: regulation of H2O2 catabolic process, regulation of hydrogen peroxide breakdown, regulation of hydrogen peroxide catabolism, regulation of hydrogen peroxide degradation, regulation of H2O2 scavenging, regulation of detoxification of H2O2, regulation of detoxification of hydrogen peroxide, regulation of hydrogen peroxide removal, regulation of hydrogen peroxide scavenging Relationships: is a type of regulation of catabolic process [GO:0009894]; is a type of regulation of hydrogen peroxide metabolic process [GO:0010310]; regulates hydrogen peroxide catabolic process [GO:0042744] Definition: Any process that modulates the frequency, rate or extent of hydrogen peroxide catabolic process.